G protein-coupled serotonin receptor complex [GO:0098666] (cellular component) Sources: GOC:TermGenie, GOC:bhm, GO_REF:0000088 Also known as: G-protein coupled serotonin receptor complex Relationships: is a type of receptor complex [GO:0043235] Definition: A protein complex that is capable of G protein-coupled serotonin receptor activity.